proteasome assembly [GO:0043248] (biological process) Regulation: regulated by GO:0090364 Also known as: proteasome complex assembly, proteasome maturation, 26S proteasome assembly Relationships: is a type of protein-containing complex assembly [GO:0065003] Definition: The aggregation, arrangement and bonding together of a mature, active proteasome complex. References: PMID:10872471 Sources: GOC:go_curators Subtypes: proteasome regulatory particle assembly [GO:0070682], proteasome core complex assembly [GO:0080129]